{
  "gene_symbol": "BBS1",
  "term_id": "GO:0061512",
  "gene": "UniProtKB:Q8NFJ9",
  "term_label": "protein localization to cilium",
  "gene_name": "Bardet-Biedl syndrome 1 protein"
}